{
  "gene": "UniProtKB:Q96LA6",
  "gene_symbol": "FCRL1",
  "term_label": "cell surface receptor signaling pathway",
  "gene_name": "Fc receptor-like protein 1",
  "term_id": "GO:0007166"
}